{
  "gene_symbol": "TRPC5OS",
  "term_id": "UNKNOWN:0003",
  "term_label": "Unknown cellular component",
  "gene": "UniProtKB:A6NMA1",
  "gene_name": "Putative uncharacterized protein TRPC5OS"
}